{
  "gene_symbol": "CDH2",
  "gene_name": "Cadherin-2",
  "term_label": "catenin complex",
  "gene": "UniProtKB:P19022",
  "term_id": "GO:0016342"
}